{
  "gene_name": "Nesprin-3",
  "gene": "UniProtKB:Q6ZMZ3",
  "gene_symbol": "SYNE3",
  "term_label": "actin filament binding",
  "term_id": "GO:0051015"
}